{
  "gene_symbol": "GRIN2C",
  "gene_name": "Glutamate receptor ionotropic, NMDA 2C",
  "term_label": "NMDA selective glutamate receptor complex",
  "gene": "UniProtKB:Q14957",
  "term_id": "GO:0017146"
}